chalcone biosynthetic process [GO:0009715] (biological process) Definition: The chemical reactions and pathways resulting in the formation of chalcone, phenyl steryl ketone or its hydroxylated derivatives. Relationships: is a type of phenylpropanoid biosynthetic process [GO:0009699]; is a type of ketone biosynthetic process [GO:0042181]; is a type of olefinic compound biosynthetic process [GO:0120255] Sources: GOC:go_curators Also known as: chalcone anabolism, chalcone biosynthesis, chalcone formation, chalcone synthesis